{
  "term_label": "double-stranded DNA binding",
  "gene_symbol": "XRCC6",
  "term_id": "GO:0003690",
  "gene_name": "X-ray repair cross-complementing protein 6",
  "gene": "UniProtKB:P12956"
}